{
  "gene": "UniProtKB:Q9NQY0",
  "gene_symbol": "BIN3",
  "term_id": "GO:0006897",
  "gene_name": "Bridging integrator 3",
  "term_label": "endocytosis"
}